sevenless signaling pathway [GO:0045500] (biological process) Definition: The series of molecular signals initiated by an extracellular ligand binding to sevenless (sev; a receptor tyrosine kinase) on the surface of a target cell, and ending with the regulation of a downstream cellular process, e.g. transcription. References: PMID:10771085 Sources: GOC:bf, GOC:signaling Also known as: sev receptor signaling pathway, sev signaling pathway, sevenless signalling pathway Relationships: is a type of cell surface receptor protein tyrosine kinase signaling pathway [GO:0007169]; is part of R7 cell fate commitment [GO:0007465] Regulation: regulated by regulation of sevenless signaling pathway [GO:0045501]; negatively regulated by GO:0045873; positively regulated by positive regulation of sevenless signaling pathway [GO:0045874]